hip joint articular cartilage development [GO:0061977] (biological process) Definition: The process whose specific outcome is the progression of hip joint articular cartilage over time, from its formation to the mature structure. References: PMID:20097540 Relationships: is a type of articular cartilage development [GO:0061975] Subtypes: femoral head articular cartilage development [GO:0061979]